protein desumoylation [GO:0016926] (biological process) Definition: The process in which a SUMO protein (small ubiquitin-related modifier) is cleaved from its target protein. Also known as: desumoylation, protein desumolation References: PMID:11265250 Sources: GOC:jl Regulation: regulated by GO:0060188; positively regulated by GO:0060189; negatively regulated by negative regulation of protein desumoylation [GO:0060190] Relationships: is a type of peptidyl-lysine modification [GO:0018205]; is a type of protein modification by small protein removal [GO:0070646]